{
  "gene": "UniProtKB:A0AVK6",
  "term_id": "GO:0000978",
  "gene_symbol": "E2F8",
  "term_label": "RNA polymerase II cis-regulatory region sequence-specific DNA binding",
  "gene_name": "Transcription factor E2F8"
}